protein insertion into plasma membrane [GO:0098737] (biological process) Definition: The process that results in the incorporation of a protein into a plasma membrane. Incorporation in this context means having some part or covalently attached group that is inserted into the the hydrophobic region of one or both bilayers. Sources: GOC:DOS Relationships: is a type of protein insertion into membrane [GO:0051205] Subtypes: protein insertion into plasma membrane raft [GO:0044859]